{
  "gene_name": "Isocitrate dehydrogenase [NAD] subunit alpha, mitochondrial",
  "gene": "UniProtKB:P50213",
  "term_label": "isocitrate metabolic process",
  "gene_symbol": "IDH3A",
  "term_id": "GO:0006102"
}